dynein-driven meiotic oscillatory nuclear movement [GO:0030989] (biological process) Definition: Oscillatory movement of the nucleus involved in meiosis I. This oscillatory movement is led by an astral microtubule array emanating from the spindle pole body, and driven by the microtubule motor cytoplasmic dynein. References: PMID:16111942, PMID:9572142 Sources: GOC:vw Also known as: HNM, horsetail movement, horsetail nuclear movement Note: Dynein-driven meiotic oscillatory nuclear movement precedes meiotic recombination. Relationships: is a type of GO:0030473; is a type of meiotic cell cycle process [GO:1903046]; is part of GO:0007127